midbrain-hindbrain boundary morphogenesis [GO:0021555] (biological process) Definition: The process in which the anatomical structure of the midbrain-hindbrain boundary is generated and organized. The midbrain-hindbrain domain of the embryonic brain is comprised of the mesencephalic vesicle and the first rhombencephalic vesicle at early somitogenesis stages. An organizing center at the boundary patterns the midbrain and hindbrain primordia of the neural plate. Also known as: MHB morphogenesis, isthmus morphogenesis Relationships: is a type of embryonic morphogenesis [GO:0048598]; is part of midbrain-hindbrain boundary development [GO:0030917] References: PMID:15541513 Sources: GOC:cls, GOC:dgh, GOC:dph, GOC:jid, GO_REF:0000021